{
  "term_label": "Unknown biological process",
  "gene_symbol": "ERH",
  "term_id": "UNKNOWN:0002",
  "gene_name": "Enhancer of rudimentary homolog",
  "gene": "UniProtKB:P84090"
}